{
  "gene": "UniProtKB:A6NH21",
  "gene_symbol": "SERINC4",
  "term_id": "GO:0016020",
  "term_label": "membrane",
  "gene_name": "Serine incorporator 4"
}